L-lysine 6-monooxygenase (NADPH) activity [GO:0047091] (molecular function) Relationships: is a type of GO:0016703; is a type of oxidoreductase activity, acting on paired donors, with incorporation or reduction of molecular oxygen, NAD(P)H as one donor, and incorporation of one atom of oxygen [GO:0016709] Also known as: L-lysine 6-monooxygenase activity, lysine N6-hydroxylase activity, L-lysine,NADPH:oxygen oxidoreductase (6-hydroxylating), lysine N(6)-hydroxylase activity Sources: EC:1.14.13.59, RHEA:23228 Definition: Catalysis of the reaction: L-lysine + NADPH + O2 = N(6)-hydroxy-L-lysine + H2O + NADP+. Note: Note that EC:1.13.12.10 was merged into this term.